{
  "term_label": "positive regulation of transcription by RNA polymerase II",
  "gene_symbol": "FUBP3",
  "gene_name": "Far upstream element-binding protein 3",
  "term_id": "GO:0045944",
  "gene": "UniProtKB:Q96I24"
}